{
  "gene": "UniProtKB:Q8NGR4",
  "term_label": "odorant binding",
  "term_id": "GO:0005549",
  "gene_symbol": "OR5C1",
  "gene_name": "Olfactory receptor 5C1"
}